transpiration [GO:0010148] (biological process) Sources: GOC:sm, ISBN:0879015322 Definition: Release of water by the plant into the air as water vapor mainly through leaves. Relationships: is a type of water transport [GO:0006833]